{
  "term_label": "proteolysis",
  "gene_symbol": "PAPPA",
  "gene_name": "Pappalysin-1",
  "gene": "UniProtKB:Q13219",
  "term_id": "GO:0006508"
}